{
  "gene_name": "Metallothionein-1M",
  "term_id": "GO:0071276",
  "gene": "UniProtKB:Q8N339",
  "term_label": "cellular response to cadmium ion",
  "gene_symbol": "MT1M"
}